melibiose:monoatomic cation symporter activity [GO:0015487] (molecular function) Definition: Enables the transfer of a solute or solutes from one side of a membrane to the other according to the reaction: melibiose(out) + monovalent cation(out) = melibiose(in) + monovalent cation(in). Subtypes: melibiose:sodium symporter activity [GO:0043887] Also known as: melibiose:cation symporter activity, melibiose:monovalent cation symporter activity, melibiose permease activity Sources: TC:2.A.2.1.1 Relationships: is a type of carbohydrate:monoatomic cation symporter activity [GO:0005402]; is a type of melibiose transmembrane transporter activity [GO:0015156]